cyclamate sulfohydrolase activity [GO:0018789] (molecular function) Sources: EC:3.10.1.2, RHEA:18481 Relationships: is a type of GO:0016826 Definition: Catalysis of the reaction: cyclohexylsulfamate + H2O = cyclohexylamine + sulfate. Also known as: cyclamate sulfamatase activity, cyclamate sulphohydrolase activity, cyclamate sulfamidase activity, cyclohexylsulfamate sulfamidase activity, cyclohexylsulfamate sulfohydrolase activity